{
  "gene_name": "Retrotransposon Gag-like protein 8B",
  "term_label": "Unknown biological process",
  "gene_symbol": "RTL8B",
  "term_id": "UNKNOWN:0002",
  "gene": "UniProtKB:Q17RB0"
}